{
  "gene_name": "Zinc finger protein 366",
  "gene": "UniProtKB:Q8N895",
  "term_id": "GO:0033147",
  "gene_symbol": "ZNF366",
  "term_label": "negative regulation of intracellular estrogen receptor signaling pathway"
}